regulation of epidermal growth factor receptor signaling pathway [GO:0042058] (biological process) Definition: Any process that modulates the frequency, rate or extent of epidermal growth factor receptor signaling pathway activity. Subtypes: negative regulation of epidermal growth factor receptor signaling pathway [GO:0042059], positive regulation of epidermal growth factor receptor signaling pathway [GO:0045742], regulation of epidermal growth factor receptor signaling pathway involved in heart process [GO:1905282] Sources: GOC:go_curators Relationships: is a type of regulation of ERBB signaling pathway [GO:1901184]; regulates epidermal growth factor receptor signaling pathway [GO:0007173] Also known as: regulation of EGF receptor signaling pathway, regulation of EGF receptor signalling pathway, regulation of EGFR signaling pathway